{
  "gene_name": "Coiled-coil domain containing 92B",
  "term_label": "Unknown cellular component",
  "term_id": "UNKNOWN:0003",
  "gene": "UniProtKB:A0A8I5KY20",
  "gene_symbol": "CCDC92B"
}